regulation of heat generation [GO:0031650] (biological process) Definition: Any process that modulates the rate or extent of heat generation. Sources: GOC:dph, GOC:mah, GOC:tb Relationships: is a type of regulation of multicellular organismal process [GO:0051239]; regulates heat generation [GO:0031649] Subtypes: regulation of fever generation [GO:0031620], GO:0031651, positive regulation of heat generation [GO:0031652]